{
  "gene_name": "POC1 centriolar protein homolog B",
  "term_id": "GO:0060271",
  "gene": "UniProtKB:Q8TC44",
  "gene_symbol": "POC1B",
  "term_label": "cilium assembly"
}